{
  "term_id": "GO:0020037",
  "gene_name": "Cytochrome P450 2C9",
  "gene_symbol": "CYP2C9",
  "gene": "UniProtKB:P11712",
  "term_label": "heme binding"
}